regulation of nerve growth factor receptor activity [GO:0051394] (biological process) Sources: GOC:ai Relationships: is a type of regulation of signaling receptor activity [GO:0010469]; regulates nerve growth factor receptor activity [GO:0010465] Definition: Any process that modulates the frequency, rate or extent of the activity of the nerve growth factor (NGF) receptor. Also known as: regulation of NGF receptor activity